epithelial cell migration involved in nephron tubule morphogenesis [GO:0072155] (biological process) Definition: The orderly movement of epithelial cells within a renal tubule that contributes to nephron tubule morphogenesis. Subtypes: epithelial cell migration involved in mesonephric nephron tubule morphogenesis [GO:0061278], epithelial cell migration involved in distal tubule morphogenesis [GO:0072157], epithelial cell migration involved in proximal tubule morphogenesis [GO:0072159], epithelial cell migration involved in metanephric nephron tubule morphogenesis [GO:0072290] Relationships: is a type of epithelial cell migration [GO:0010631]; is a type of cell migration involved in kidney development [GO:0035787]; is part of GO:0072078 Sources: GOC:mtg_kidney_jan10